phosphatidylinositol deacylase activity [GO:0050185] (molecular function) Also known as: 1-phosphatidyl-D-myo-inositol 2-acylhydrolase activity, phosphatidylinositol phospholipase A2 activity Sources: EC:3.1.1.52, RHEA:18001 Definition: Catalysis of the reaction: 1-phosphatidyl-1D-myo-inositol + H2O = 1-acyl-sn-glycero-3-phospho-D-myo-inositol + a carboxylate + H+. Relationships: is a type of GO:0052689